L-leucine biosynthetic process [GO:0009098] (biological process) Definition: The chemical reactions and pathways resulting in the formation of L-leucine, 2-amino-4-methylpentanoic acid. Sources: GOC:ai Also known as: leucine biosynthetic process, L-leucine anabolism, L-leucine biosynthesis, L-leucine formation, L-leucine synthesis Relationships: is a type of L-leucine metabolic process [GO:0006551]; is a type of pyruvate family amino acid biosynthetic process [GO:0009079]; is a type of branched-chain amino acid biosynthetic process [GO:0009082] Regulation: regulated by regulation of L-leucine biosynthetic process [GO:2001276]; negatively regulated by GO:2001277; positively regulated by positive regulation of L-leucine biosynthetic process [GO:2001278]